{
  "gene_symbol": "IFIT1B",
  "gene": "UniProtKB:Q5T764",
  "term_id": "GO:0140374",
  "gene_name": "Interferon-induced protein with tetratricopeptide repeats 1B",
  "term_label": "antiviral innate immune response"
}